venous blood vessel development [GO:0060841] (biological process) Sources: GOC:dph, GOC:sdb_2009, GOC:tb Definition: The progression of the venous blood vessel over time from its initial formation to the mature structure. Venous blood vessels carry blood back to the heart after the capillary bed. Relationships: is_a blood vessel development [GO:0001568]